{
  "gene_name": "Putative uncharacterized protein FLJ37218",
  "term_label": "Unknown cellular component",
  "term_id": "UNKNOWN:0003",
  "gene": "UniProtKB:Q8N1Y9",
  "gene_symbol": "Q8N1Y9"
}